{
  "gene_symbol": "LILRA6",
  "gene_name": "Leukocyte immunoglobulin-like receptor subfamily A member 6",
  "term_id": "GO:0032396",
  "term_label": "inhibitory MHC class I receptor activity",
  "gene": "UniProtKB:Q6PI73"
}